{
  "gene_name": "Olfactory receptor 6K3",
  "term_label": "odorant binding",
  "term_id": "GO:0005549",
  "gene": "UniProtKB:Q8NGY3",
  "gene_symbol": "OR6K3"
}